intracellular organelle lumen [GO:0070013] (CC) Sources: GOC:mah Relationships: is a type of organelle lumen [GO:0043233]; is part of intracellular organelle [GO:0043229] Subtypes: GO:0005759, vacuolar lumen [GO:0005775], endoplasmic reticulum lumen [GO:0005788], Golgi lumen [GO:0005796], GO:0031096, endosome lumen [GO:0031904], microbody lumen [GO:0031907], GO:0031970, nuclear lumen [GO:0031981], acidocalcisome lumen [GO:0033985], hydrogenosome lumen [GO:0034492], microneme lumen [GO:0034494], gut granule lumen [GO:0044842], cytoplasmic vesicle lumen [GO:0060205], endocytic vesicle lumen [GO:0071682], multivesicular body, internal vesicle lumen [GO:0097489], magnetosome lumen [GO:0110145], tertiary granule lumen [GO:1904724], ficolin-1-rich granule lumen [GO:1904813] Definition: An organelle lumen that is part of an intracellular organelle.